{
  "gene_name": "Carcinoembryonic antigen-related cell adhesion molecule 5",
  "gene": "UniProtKB:P06731",
  "term_id": "GO:0007156",
  "term_label": "homophilic cell-cell adhesion",
  "gene_symbol": "CEACAM5"
}